{
  "term_id": "GO:0035456",
  "term_label": "response to interferon-beta",
  "gene_symbol": "C9JQL5",
  "gene": "UniProtKB:C9JQL5",
  "gene_name": "Putative dispanin subfamily A member 2d"
}